alpha-N-acetylgalactosaminide alpha-2,6-sialyltransferase activity [GO:0001665] (molecular function) Definition: Catalysis of the reaction: CMP-N-acetylneuraminate + glycano-(1->3)-(N-acetyl-alpha-D-galactosaminyl)-glycoprotein = CMP + glycano-[(2->6)-alpha-N-acetylneuraminyl]-(N-acetyl-D-galactosaminyl)-glycoprotein. Sources: EC:2.4.3.3 Also known as: GalNAc alpha-2,6-sialyltransferase I activity Relationships: is_a sialyltransferase activity [GO:0008373]